{
  "term_id": "GO:0005737",
  "gene": "UniProtKB:Q7Z4G4",
  "term_label": "cytoplasm",
  "gene_symbol": "TRMT11",
  "gene_name": "tRNA (guanine(10)-N2)-methyltransferase homolog"
}